{
  "term_id": "UNKNOWN:0002",
  "gene_symbol": "FUT3",
  "gene_name": "3-galactosyl-N-acetylglucosaminide 4-alpha-L-fucosyltransferase FUT3",
  "term_label": "Unknown biological process",
  "gene": "UniProtKB:P21217"
}